{
  "gene_symbol": "TIFA",
  "gene": "UniProtKB:Q96CG3",
  "gene_name": "TRAF-interacting protein with FHA domain-containing protein A",
  "term_label": "Unknown molecular function",
  "term_id": "UNKNOWN:0001"
}